{
  "term_id": "GO:0006508",
  "term_label": "proteolysis",
  "gene_name": "Puromycin-sensitive aminopeptidase-like protein",
  "gene": "UniProtKB:A6NEC2",
  "gene_symbol": "NPEPPSL1"
}